{
  "term_id": "UNKNOWN:0002",
  "gene_name": "Hyaluronan mediated motility receptor",
  "term_label": "Unknown biological process",
  "gene": "UniProtKB:O75330",
  "gene_symbol": "HMMR"
}